{
  "gene_name": "Protein lin-28 homolog B",
  "term_id": "GO:0005634",
  "gene_symbol": "LIN28B",
  "gene": "UniProtKB:Q6ZN17",
  "term_label": "nucleus"
}